{
  "term_label": "phosphatidylcholine biosynthetic process",
  "gene_name": "Phosphatidylethanolamine N-methyltransferase",
  "gene_symbol": "PEMT",
  "gene": "UniProtKB:Q9UBM1",
  "term_id": "GO:0006656"
}